AUG codon-amino acid adaptor activity [GO:0033436] (molecular function) Also known as: ATG codon-amino acid adaptor activity, initiator methionine tRNA, methionine tRNA Note: Note that in the standard genetic code, ATG codes for methionine, and is the initiator codon. Definition: A triplet codon-amino acid adaptor activity that recognizes an AUG codon. Sources: GOC:mah Relationships: is a type of GO:0030533